{
  "gene": "UniProtKB:Q9NYG8",
  "term_label": "potassium ion transmembrane transport",
  "term_id": "GO:0071805",
  "gene_name": "Potassium channel subfamily K member 4",
  "gene_symbol": "KCNK4"
}